{
  "gene_symbol": "SARDH",
  "gene_name": "Sarcosine dehydrogenase, mitochondrial",
  "term_id": "GO:0005737",
  "gene": "UniProtKB:Q9UL12",
  "term_label": "cytoplasm"
}